{
  "gene_symbol": "PSD",
  "term_id": "GO:0005085",
  "gene_name": "PH and SEC7 domain-containing protein 1",
  "term_label": "guanyl-nucleotide exchange factor activity",
  "gene": "UniProtKB:A5PKW4"
}